2,5-dioxovalerate dehydrogenase (NAD+) activity [GO:0044104] (molecular function) References: PMID:16835232, PMID:17202142 Relationships: is a type of GO:0016620 Definition: Catalysis of the reaction: 2,5-dioxopentanoate + NAD+ + H2O = 2-oxoglutarate + NADH + H+. Also known as: 2,5-dioxopentanoate dehydrogenase (NAD+) activity, 2,5-dioxopentanoate:NAD+ 5-oxidoreductase activity